{
  "gene": "UniProtKB:Q9UNX3",
  "term_label": "ribosomal large subunit biogenesis",
  "gene_name": "Ribosomal protein uL24-like",
  "gene_symbol": "RPL26L1",
  "term_id": "GO:0042273"
}